{
  "gene_name": "Centrin-2",
  "term_id": "GO:0007099",
  "term_label": "centriole replication",
  "gene": "UniProtKB:P41208",
  "gene_symbol": "CETN2"
}